circadian sleep/wake cycle, non-REM sleep [GO:0042748] (biological process) Definition: All sleep stages in the circadian sleep/wake cycle other than REM sleep. These stages are characterized by a slowing of brain waves and other physiological functions. References: PMID:33537937 Sources: GOC:jl Relationships: is a type of GO:0022410; is part of circadian sleep/wake cycle, sleep [GO:0050802] Regulation: negatively regulated by negative regulation of circadian sleep/wake cycle, non-REM sleep [GO:0042323]; regulated by GO:0045188; positively regulated by GO:0046010